{
  "gene_name": "DnaJ homolog subfamily B member 8",
  "gene": "UniProtKB:Q8NHS0",
  "term_id": "GO:0044183",
  "gene_symbol": "DNAJB8",
  "term_label": "protein folding chaperone"
}